UDP-N-acetylmuramoyl-L-alanyl-D-glutamyl-meso-2,6-diaminopimelyl-D-alanyl-D-alanine:undecaprenyl-phosphate transferase activity [GO:0051992] (molecular function) Definition: Catalysis of the reaction: di-trans,octa-cis-undecaprenyl phosphate + UDP-N-acetyl-alpha-D-muramoyl-L-alanyl-gamma-D-glutamyl-meso-2,6-diaminopimeloyl-D-alanyl-D-alanine = di-trans-octa-cis-undecaprenyl diphospho-N-acetyl-alpha-D-muramoyl-L-alanyl-D-glutamyl-meso-2,6-diaminopimeloyl-D-alanyl-D-alanine + UMP. Sources: RHEA:28386 Note: Note that EC classifies 'UDP-N-acetylmuramoyl-L-alanyl-D-glutamyl-meso-2,6-diaminopimelyl-D-alanyl-D-alanine:undecaprenyl-phosphate transferase activity ; GO:0051992' and 'phospho-N-acetylmuramoyl-pentapeptide-transferase activity ; GO:0008963' under the same EC number, EC:2.7.8.13. Relationships: is a type of phosphotransferase activity, for other substituted phosphate groups [GO:0016780]